amino acid:monoatomic cation symporter activity [GO:0005416] (MF) Definition: Enables the transfer of a solute or solutes from one side of a membrane to the other according to the reaction: amino acid(out) + cation(out) = amino acid(in) + cation(in). Also known as: amino acid:cation symporter activity, cation/amino acid symporter activity, cation:amino acid symporter activity Relationships: is a type of GO:0015171; is_a solute:monoatomic cation symporter activity [GO:0015294] Subtypes: amino acid:proton symporter activity [GO:0005280], GO:0005283, amino acid:potassium symporter activity [GO:0017032] Sources: GOC:ai